{
  "term_id": "GO:0000981",
  "term_label": "DNA-binding transcription factor activity, RNA polymerase II-specific",
  "gene": "UniProtKB:O95625",
  "gene_name": "Zinc finger and BTB domain-containing protein 11",
  "gene_symbol": "ZBTB11"
}